box H/ACA RNP complex [GO:0072588] (cellular component) Subtypes: box H/ACA snoRNP complex [GO:0031429], box H/ACA scaRNP complex [GO:0072589], GO:0090661 Relationships: is a type of sno(s)RNA-containing ribonucleoprotein complex [GO:0005732] Definition: A ribonucleoprotein complex that contains an RNA of the box H/ACA type and the four core proteins dyskerin, NOP10, NHP2, and GAR1 (human protein nomenclature). RNA pseudouridylation (isomerization of uridine to pseudouridine) is the major, and most likely the ancestral, function of H/ACA RNPs. Pseudouridylation targets include both large and small ribosomal RNAs (rRNAs), and small nuclear RNA (U2 snRNA). In addition to these catalytic H/ACA RNPs, a less abundant but more diverse class of structural H/ACA RNPs exists, which does not have pseudouridylation activity. These include the vertebrate telomerase RNP complex. Also known as: sRNP complex, box H/ACA snoRNP pseudouridylase complex References: PMID:17284456, PMID:20227365, PMID:25590339 Sources: GOC:BHF, GOC:BHF_telomerase, GOC:jbu, GOC:krc, GOC:mah